{
  "term_id": "GO:0033787",
  "term_label": "cyanocobalamin reductase (cyanide-eliminating) (NADP+) activity",
  "gene_symbol": "MMACHC",
  "gene": "UniProtKB:Q9Y4U1",
  "gene_name": "Cyanocobalamin reductase _ alkylcobalamin dealkylase"
}